{
  "gene_name": "Copine-5",
  "gene_symbol": "CPNE5",
  "term_label": "cellular response to calcium ion",
  "term_id": "GO:0071277",
  "gene": "UniProtKB:Q9HCH3"
}